{
  "term_label": "ATP-dependent peptidase activity",
  "gene": "UniProtKB:Q96TA2",
  "gene_name": "ATP-dependent zinc metalloprotease YME1L1",
  "gene_symbol": "YME1L1",
  "term_id": "GO:0004176"
}